{
  "gene": "UniProtKB:Q58EX2",
  "gene_name": "Protein sidekick-2",
  "gene_symbol": "SDK2",
  "term_label": "homophilic cell-cell adhesion",
  "term_id": "GO:0007156"
}